phytol biosynthetic process [GO:0033520] (biological process) Relationships: is a type of diterpenoid biosynthetic process [GO:0016102]; is_a phytol metabolic process [GO:0033306]; is a type of GO:0034309; is a type of fatty alcohol biosynthetic process [GO:1903175] Definition: The chemical reactions and pathways resulting in the formation of phytol, (2E,7R,11R)-3,7,11,15-tetramethylhexadec-2-en-1-ol. Sources: GOC:mah Also known as: phytol anabolism, phytol biosynthesis, phytol formation, phytol synthesis Subtypes: phytol salvage [GO:0033307] Regulation: regulated by regulation of phytol biosynthetic process [GO:1904963]; positively regulated by positive regulation of phytol biosynthetic process [GO:1904964]